regulation of opioid receptor signaling pathway [GO:2000474] (biological process) Also known as: regulation of opioid receptor signalling pathway Sources: GOC:obol Subtypes: regulation of adenylate cyclase-inhibiting opioid receptor signaling pathway [GO:1900729], negative regulation of opioid receptor signaling pathway [GO:2000475], positive regulation of opioid receptor signaling pathway [GO:2000476] Relationships: is a type of GO:0008277; regulates G protein-coupled opioid receptor signaling pathway [GO:0038003] Definition: Any process that modulates the frequency, rate or extent of opioid receptor signaling pathway.